{
  "term_id": "GO:0005654",
  "gene": "UniProtKB:Q5TC79",
  "gene_name": "Zinc finger and BTB domain-containing protein 37",
  "term_label": "nucleoplasm",
  "gene_symbol": "ZBTB37"
}